{
  "term_label": "vitamin D catabolic process",
  "gene_name": "1,25-dihydroxyvitamin D(3) 24-hydroxylase, mitochondrial",
  "gene": "UniProtKB:Q07973",
  "gene_symbol": "CYP24A1",
  "term_id": "GO:0042369"
}